negative regulation of store-operated calcium entry [GO:0106128] (biological process) Relationships: is a type of GO:0051926; is a type of regulation of store-operated calcium entry [GO:2001256]; negatively regulates store-operated calcium entry [GO:0002115] References: PMID:23447642 Sources: GOC:BHF, GOC:BHF_miRNA, GOC:rph Definition: Any process that stops, prevents or reduces the frequency, rate or extent of store-operated calcium entry.